positive regulation of trehalose catabolic process [GO:1901319] (biological process) Definition: Any process that activates or increases the frequency, rate or extent of trehalose catabolic process. Sources: GOC:TermGenie Relationships: is a type of positive regulation of catabolic process [GO:0009896]; is a type of regulation of carbohydrate catabolic process [GO:0043470]; is_a positive regulation of carbohydrate metabolic process [GO:0045913]; is a type of GO:0090062; positively regulates trehalose catabolic process [GO:0005993] Also known as: activation of mycose catabolic process, activation of mycose catabolism, activation of mykose catabolic process, activation of mykose catabolism, activation of trehalose breakdown, activation of trehalose catabolism, activation of trehalose degradation, positive regulation of mycose catabolic process, positive regulation of mycose catabolism, positive regulation of mykose catabolic process, positive regulation of mykose catabolism, positive regulation of trehalose breakdown, positive regulation of trehalose catabolism, positive regulation of trehalose degradation, up regulation of mycose catabolic process, up regulation of mycose catabolism, up regulation of mykose catabolic process, up regulation of mykose catabolism, up regulation of trehalose breakdown, up regulation of trehalose catabolic process, up regulation of trehalose catabolism, up regulation of trehalose degradation, up-regulation of mycose catabolic process, up-regulation of mycose catabolism, up-regulation of mykose catabolic process, up-regulation of mykose catabolism, up-regulation of trehalose breakdown, up-regulation of trehalose catabolic process, up-regulation of trehalose catabolism, up-regulation of trehalose degradation, upregulation of mycose catabolic process, upregulation of mycose catabolism, upregulation of mykose catabolic process, upregulation of mykose catabolism, upregulation of trehalose breakdown, upregulation of trehalose catabolic process, upregulation of trehalose catabolism, upregulation of trehalose degradation, activation of trehalose catabolic process